{
  "gene_symbol": "CD47",
  "term_label": "positive regulation of cell-cell adhesion",
  "gene": "UniProtKB:Q08722",
  "term_id": "GO:0022409",
  "gene_name": "Leukocyte surface antigen CD47"
}